{
  "gene": "UniProtKB:Q15911",
  "term_label": "DNA-binding transcription factor activity, RNA polymerase II-specific",
  "gene_symbol": "ZFHX3",
  "term_id": "GO:0000981",
  "gene_name": "Zinc finger homeobox protein 3"
}